{
  "gene_name": "Amyloid beta precursor protein binding family B member 1",
  "term_label": "DNA damage response",
  "gene": "UniProtKB:O00213",
  "term_id": "GO:0006974",
  "gene_symbol": "APBB1"
}